sesquiterpene synthase activity [GO:0010334] (molecular function) Subtypes: vetispiradiene synthase activity [GO:0034003], germacrene-A synthase activity [GO:0034005], amorpha-4,11-diene synthase activity [GO:0034006], trichodiene synthase activity [GO:0045482], GO:0045483, (+)-delta-cadinene synthase activity [GO:0047461], pentalenene synthase activity [GO:0050467], germacrene-D synthase activity [GO:0052577], alpha-farnesene synthase activity [GO:0052578], (2S,3R,6S,9S)-(-)-protoillud-7-ene synthase activity [GO:0061923], (-)-E-beta-caryophyllene synthase activity [GO:0080016], alpha-humulene synthase activity [GO:0080017], (3S)-(+)-asterisca-2(9),6-diene synthase activity [GO:0120086] Sources: GOC:tair_curators Relationships: is a type of terpene synthase activity [GO:0010333] Definition: Catalysis of the reaction: trans,trans-farnesyl diphosphate = a sesquiterpene + diphosphate. Sesquiterpenes are terpenes containing three isoprene units, i.e. 15 carbons.